{
  "term_id": "GO:0043130",
  "term_label": "ubiquitin binding",
  "gene_symbol": "UBXN11",
  "gene": "UniProtKB:Q5T124",
  "gene_name": "UBX domain-containing protein 11"
}